{
  "term_id": "GO:0052816",
  "term_label": "long-chain fatty acyl-CoA hydrolase activity",
  "gene_symbol": "PLA2G6",
  "gene_name": "85_88 kDa calcium-independent phospholipase A2",
  "gene": "UniProtKB:O60733"
}